{
  "gene": "UniProtKB:Q13207",
  "gene_name": "T-box transcription factor TBX2",
  "term_label": "nucleus",
  "gene_symbol": "TBX2",
  "term_id": "GO:0005634"
}